{
  "gene_name": "Protein S100-A2",
  "gene": "UniProtKB:P29034",
  "term_id": "UNKNOWN:0003",
  "gene_symbol": "S100A2",
  "term_label": "Unknown cellular component"
}